thymidine kinase activity [GO:0004797] (molecular function) Sources: EC:2.7.1.21 Definition: Catalysis of the reaction: ATP + thymidine = ADP + thymidine 5'-phosphate. Relationships: is a type of GO:0019136 Also known as: 2'-deoxythymidine kinase activity, ATP:thymidine 5'-phosphotransferase activity, deoxythymidine kinase (phosphorylating), thymidine kinase (phosphorylating)